{
  "gene_symbol": "SEPTIN5",
  "term_label": "synaptic vesicle",
  "gene": "UniProtKB:Q99719",
  "gene_name": "Septin-5",
  "term_id": "GO:0008021"
}